{
  "term_id": "GO:0005634",
  "term_label": "nucleus",
  "gene_symbol": "TDRP",
  "gene": "UniProtKB:Q86YL5",
  "gene_name": "Testis development-related protein"
}